{
  "gene": "UniProtKB:Q49AM3",
  "gene_name": "Tetratricopeptide repeat protein 31",
  "gene_symbol": "TTC31",
  "term_id": "UNKNOWN:0003",
  "term_label": "Unknown cellular component"
}